{
  "term_id": "GO:0050832",
  "gene": "UniProtKB:Q8TDE3",
  "term_label": "defense response to fungus",
  "gene_symbol": "RNASE8",
  "gene_name": "Ribonuclease 8"
}